{
  "gene": "UniProtKB:P0CJ68",
  "gene_name": "Humanin-like 1",
  "term_label": "negative regulation of execution phase of apoptosis",
  "gene_symbol": "MTRNR2L1",
  "term_id": "GO:1900118"
}